{
  "term_id": "GO:0045095",
  "term_label": "keratin filament",
  "gene_symbol": "KRT33A",
  "gene_name": "Keratin, type I cuticular Ha3-I",
  "gene": "UniProtKB:O76009"
}